{
  "gene_name": "Olfactory receptor",
  "term_label": "Unknown cellular component",
  "term_id": "UNKNOWN:0003",
  "gene": "UniProtKB:A0A126GWI2",
  "gene_symbol": "OR2A25"
}